{
  "gene_name": "Zinc finger protein 641",
  "term_id": "GO:0006357",
  "gene": "UniProtKB:Q96N77",
  "gene_symbol": "ZNF641",
  "term_label": "regulation of transcription by RNA polymerase II"
}